{
  "gene": "UniProtKB:Q8WY36",
  "gene_name": "HMG box transcription factor BBX",
  "term_id": "GO:0005634",
  "term_label": "nucleus",
  "gene_symbol": "BBX"
}